{
  "gene_symbol": "COBL",
  "gene": "UniProtKB:O75128",
  "term_id": "GO:0044295",
  "term_label": "axonal growth cone",
  "gene_name": "Protein cordon-bleu"
}